{
  "term_id": "GO:0034198",
  "gene_symbol": "GCN1",
  "gene_name": "Stalled ribosome sensor GCN1",
  "term_label": "cellular response to amino acid starvation",
  "gene": "UniProtKB:Q92616"
}